molecular sensor activity [GO:0140299] (MF) Also known as: small molecular sensor activity, small molecule sensing activity, small molecule sensor activity References: PMID:26328879 Definition: Binding to a molecule and eliciting a change in the protein's activity in response to the intracellular level of that molecule. Relationships: is a type of molecular function regulator activity [GO:0098772] Subtypes: phosphorelay sensor kinase activity [GO:0000155], GO:0005034, oxygen sensor activity [GO:0019826], nitric oxide sensor activity [GO:0035991], carbon monoxide sensor activity [GO:0070027], GO:0106254, membrane curvature sensor activity [GO:0140090], GO:0140442, DNA damage sensor activity [GO:0140612], metal ion sensor activity [GO:0140784], amino acid sensor activity [GO:0140785], GO:0141089, stalled ribosome sensor activity [GO:0170011], inositol pyrophosphate sensor activity [GO:0180043]